{
  "gene_symbol": "SETD3",
  "term_label": "positive regulation of transcription by RNA polymerase II",
  "gene": "UniProtKB:Q86TU7",
  "gene_name": "Actin-histidine N-methyltransferase",
  "term_id": "GO:0045944"
}